{
  "gene": "UniProtKB:Q9Y275",
  "gene_name": "Tumor necrosis factor ligand superfamily member 13B",
  "term_id": "GO:0005615",
  "gene_symbol": "TNFSF13B",
  "term_label": "extracellular space"
}